cellular response to diterpene [GO:1904630] (biological process) Definition: Any process that results in a change in state or activity of a cell (in terms of movement, secretion, enzyme production, gene expression, etc.) as a result of a diterpene stimulus. References: PMID:19765580 Sources: GOC:TermGenie, GO_REF:0000071 Relationships: is a type of cellular response to lipid [GO:0071396]; is_a response to diterpene [GO:1904629]